{
  "gene_symbol": "HMGCLL1",
  "term_id": "GO:0006552",
  "term_label": "L-leucine catabolic process",
  "gene": "UniProtKB:Q8TB92",
  "gene_name": "3-hydroxy-3-methylglutaryl-CoA lyase, cytoplasmic"
}